{
  "gene_name": "All trans-polyprenyl-diphosphate synthase PDSS2",
  "term_label": "mitochondrion",
  "term_id": "GO:0005739",
  "gene": "UniProtKB:Q86YH6",
  "gene_symbol": "PDSS2"
}